{
  "gene": "UniProtKB:Q30KR1",
  "term_id": "GO:0005615",
  "gene_name": "Putative beta-defensin 109B",
  "gene_symbol": "DEFB109B",
  "term_label": "extracellular space"
}